myosin XVI complex [GO:0031486] (cellular component) References: PMID:11294886, PMID:32451869 Definition: A myosin complex containing a class XVI myosin heavy chains and associated light chains; myosin XVI heavy chains contain ankyrin repeat. Relationships: is a type of GO:0016461